{
  "gene": "UniProtKB:Q96BZ4",
  "gene_symbol": "PLD4",
  "gene_name": "5'-3' exonuclease PLD4",
  "term_id": "GO:0012505",
  "term_label": "endomembrane system"
}